myosin III binding [GO:0031473] (molecular function) Definition: Binding to a class III myosin; myosin III is monomeric and has an N terminal kinase domain. Sources: GOC:mah Relationships: is a type of GO:0017022